{
  "gene_symbol": "KIAA0586",
  "gene": "UniProtKB:Q9BVV6",
  "gene_name": "Protein TALPID3",
  "term_id": "GO:0007224",
  "term_label": "smoothened signaling pathway"
}